{
  "gene": "UniProtKB:Q9H3D4",
  "term_label": "chromatin",
  "gene_name": "Tumor protein 63",
  "gene_symbol": "TP63",
  "term_id": "GO:0000785"
}